3'(2'),5'-bisphosphate nucleotidase activity [GO:0008441] (molecular function) Also known as: 3'(2'),5' bisphosphate nucleotidase activity, 3'(2'),5'-bisphosphonucleoside 3'(2')-phosphohydrolase activity, 3'-phosphoadenylylsulfate 3'-phosphatase activity, DPNPase activity, adenosine-3'(2'),5'-bisphosphate 3'(2')-phosphohydrolase activity, phosphoadenylate 3'-nucleotidase activity Sources: EC:3.1.3.7 Definition: Catalysis of the reaction: adenosine 3',5'-bisphosphate + H2O = adenosine 5'-phosphate + phosphate. Relationships: is a type of nucleotidase activity [GO:0008252]